{
  "term_label": "cell surface receptor signaling pathway",
  "gene_name": "T cell receptor beta variable 6-8",
  "term_id": "GO:0007166",
  "gene_symbol": "TRBV6-8",
  "gene": "UniProtKB:A0A0A6YYG3"
}